negative regulation of metallopeptidase activity [GO:1905049] (biological process) Definition: Any process that stops, prevents or reduces the frequency, rate or extent of metallopeptidase activity. Also known as: down regulation of metallopeptidase activity, down-regulation of metallopeptidase activity, downregulation of metallopeptidase activity, down regulation of metalloprotease activity, down regulation of metalloproteinase activity, down-regulation of metalloprotease activity, down-regulation of metalloproteinase activity, downregulation of metalloprotease activity, downregulation of metalloproteinase activity, inhibition of metallopeptidase activity, inhibition of metalloprotease activity, inhibition of metalloproteinase activity, negative regulation of metalloprotease activity, negative regulation of metalloproteinase activity References: PMID:26473732 Sources: GOC:TermGenie, GO_REF:0000059 Relationships: is a type of GO:0010466; is a type of regulation of metallopeptidase activity [GO:1905048]; negatively regulates metallopeptidase activity [GO:0008237]